{
  "term_id": "UNKNOWN:0001",
  "gene": "UniProtKB:Q96PC5",
  "gene_symbol": "MIA2",
  "term_label": "Unknown molecular function",
  "gene_name": "Melanoma inhibitory activity protein 2"
}